{
  "term_label": "Unknown cellular component",
  "gene_name": "T cell receptor beta joining 2-6",
  "term_id": "UNKNOWN:0003",
  "gene_symbol": "TRBJ2-6",
  "gene": "UniProtKB:A0A0A0MT70"
}